{
  "term_label": "Golgi membrane",
  "term_id": "GO:0000139",
  "gene": "UniProtKB:Q6ZMB0",
  "gene_name": "Acetylgalactosaminyl-O-glycosyl-glycoprotein beta-1,3-N-acetylglucosaminyltransferase",
  "gene_symbol": "B3GNT6"
}